{
  "term_id": "GO:0000981",
  "term_label": "DNA-binding transcription factor activity, RNA polymerase II-specific",
  "gene_name": "Forkhead box protein K1",
  "gene_symbol": "FOXK1",
  "gene": "UniProtKB:P85037"
}